pyrimidine ribonucleotide salvage [GO:0010138] (biological process) Relationships: is_a GO:0009220; is a type of GO:0032262 Subtypes: CMP salvage [GO:0006238], UMP salvage [GO:0044206], GO:0044211 Definition: The pathway by which pyrimidine bases or pyrimidine ribonucleosides from pyrimidine nucleotide breakdown are converted back to pyrimidine ribonucleotides. The salvage pathway is important where there is no de novo pyrimidine nucleotide biosynthesis. Sources: GOC:pz